{
  "term_label": "potassium ion transmembrane transport",
  "gene_name": "Potassium_sodium hyperpolarization-activated cyclic nucleotide-gated channel 4",
  "gene": "UniProtKB:Q9Y3Q4",
  "gene_symbol": "HCN4",
  "term_id": "GO:0071805"
}